{
  "term_label": "mitochondrial matrix",
  "gene_symbol": "CLPX",
  "term_id": "GO:0005759",
  "gene_name": "ATP-dependent Clp protease ATP-binding subunit clpX-like, mitochondrial",
  "gene": "UniProtKB:O76031"
}